{
  "term_id": "GO:0031213",
  "gene": "UniProtKB:Q96T23",
  "term_label": "RSF complex",
  "gene_symbol": "RSF1",
  "gene_name": "Remodeling and spacing factor 1"
}